{
  "gene_symbol": "TASOR",
  "term_id": "GO:0045814",
  "gene_name": "Protein TASOR",
  "term_label": "negative regulation of gene expression, epigenetic",
  "gene": "UniProtKB:Q9UK61"
}